{
  "gene_symbol": "MICALL1",
  "gene": "UniProtKB:Q8N3F8",
  "gene_name": "MICAL-like protein 1",
  "term_id": "GO:0005886",
  "term_label": "plasma membrane"
}